{
  "gene_name": "Forkhead box protein N4",
  "term_id": "GO:0006355",
  "gene_symbol": "FOXN4",
  "term_label": "regulation of DNA-templated transcription",
  "gene": "UniProtKB:Q96NZ1"
}